regulation of neurotrophin production [GO:0032899] (biological process) Sources: GOC:mah Definition: Any process that modulates the frequency, rate, or extent of production of a neurotrophin. Relationships: is a type of regulation of multicellular organismal process [GO:0051239]; regulates neurotrophin production [GO:0032898] Subtypes: negative regulation of neurotrophin production [GO:0032900], positive regulation of neurotrophin production [GO:0032901], GO:0032903